{
  "gene_name": "NADH dehydrogenase [ubiquinone] 1 alpha subcomplex subunit 13",
  "term_label": "Unknown molecular function",
  "gene_symbol": "NDUFA13",
  "term_id": "UNKNOWN:0001",
  "gene": "UniProtKB:Q9P0J0"
}